{
  "gene_symbol": "GUCY1A2",
  "gene": "UniProtKB:P33402",
  "gene_name": "Guanylate cyclase soluble subunit alpha-2",
  "term_id": "GO:0004383",
  "term_label": "guanylate cyclase activity"
}